{
  "term_label": "RNA helicase activity",
  "gene_symbol": "SKIC2",
  "term_id": "GO:0003724",
  "gene_name": "Superkiller complex protein 2",
  "gene": "UniProtKB:Q15477"
}